symbiont-mediated suppression of host G protein-coupled receptor signal transduction [GO:0075120] (biological process) Definition: A process in which a symbiont interferes with, inhibits or disrupts a G protein-coupled receptor signal transduction in its host organism. The host is defined as the larger of the organisms involved in a symbiotic interaction. Subtypes: symbiont-mediated suppression of host chemokine signal transduction pathway [GO:0141135] Relationships: is a type of GO:0052029; is a type of symbiont-mediated perturbation of host G protein-coupled receptor signal transduction pathway [GO:0075118] References: PMID:17562776, PMID:23027529 Sources: GOC:pamgo_curators Also known as: disruption of host G protein-coupled receptor signal transduction, negative regulation by symbiont of host G protein-coupled receptor signal transduction, negative regulation by symbiont of host G-protein coupled receptor protein signal transduction, suppression by symbiont of host G protein-coupled receptor signal transduction, negative regulation by symbiont of host signal transduction mediated by G-protein alpha subunit, negative regulation by symbiont of host signal transduction mediated by G-protein beta subunit, negative regulation by symbiont of host signal transduction mediated by G-protein gamma subunit